{
  "gene_symbol": "Q8NAQ8",
  "gene": "UniProtKB:Q8NAQ8",
  "gene_name": "Putative uncharacterized protein FLJ34945",
  "term_id": "UNKNOWN:0003",
  "term_label": "Unknown cellular component"
}